{
  "term_id": "GO:0047444",
  "term_label": "N-acylneuraminate-9-phosphate synthase activity",
  "gene": "UniProtKB:Q9NR45",
  "gene_symbol": "NANS",
  "gene_name": "Sialic acid synthase"
}